kaempferol 4'-O-methyltransferase activity [GO:0033803] (MF) Sources: RHEA:15105 Relationships: is a type of O-methyltransferase activity [GO:0008171]; is a type of S-adenosylmethionine-dependent methyltransferase activity [GO:0008757] Definition: Catalysis of the reaction: S-adenosyl-L-methionine + kaempferol = S-adenosyl-L-homocysteine + H+ + kaempferide. Also known as: F 4'-OMT, S-adenosyl-L-methionine:flavonoid 4'-O-methyltransferase activity, S-adenosyl-L-methionine:kaempferol 4'-O-methyltransferase activity